{
  "term_label": "SNARE binding",
  "term_id": "GO:0000149",
  "gene_symbol": "VTI1B",
  "gene_name": "Vesicle transport through interaction with t-SNAREs homolog 1B",
  "gene": "UniProtKB:Q9UEU0"
}